positive regulation of antibacterial peptide secretion [GO:0002799] (biological process) Relationships: is a type of positive regulation of antimicrobial peptide secretion [GO:0002796]; is a type of regulation of antibacterial peptide secretion [GO:0002797]; is_a positive regulation of antibacterial peptide production [GO:0002803]; positively regulates antibacterial peptide secretion [GO:0002779] Also known as: up regulation of antibacterial peptide secretion, up-regulation of antibacterial peptide secretion, upregulation of antibacterial peptide secretion, activation of antibacterial peptide secretion, stimulation of antibacterial peptide secretion Sources: GOC:add Definition: Any process that activates or increases the frequency, rate, or extent of antibacterial peptide secretion.